{
  "term_id": "GO:0000727",
  "term_label": "double-strand break repair via break-induced replication",
  "gene_symbol": "CDC45",
  "gene": "UniProtKB:O75419",
  "gene_name": "Cell division control protein 45 homolog"
}